protein transport across periplasmic space [GO:0072322] (biological process) Also known as: chaperone-mediated protein transport across periplasmic space Definition: The directed movement of proteins from the plasma membrane across the periplasmic space to the outer membrane or cell wall. Relationships: is a type of GO:0015031; has part protein carrier chaperone [GO:0140597] References: PMID:20378773 Sources: GOC:mah